{
  "term_label": "Unknown cellular component",
  "gene_symbol": "A8MX80",
  "gene": "UniProtKB:A8MX80",
  "gene_name": "Putative UPF0607 protein ENSP00000383144",
  "term_id": "UNKNOWN:0003"
}